{
  "gene_symbol": "CAMKV",
  "gene": "UniProtKB:Q8NCB2",
  "term_id": "GO:0045202",
  "gene_name": "CaM kinase-like vesicle-associated protein",
  "term_label": "synapse"
}